{
  "term_label": "immune response",
  "gene_symbol": "IGKV1D-16",
  "gene_name": "Immunoglobulin kappa variable 1D-16",
  "term_id": "GO:0006955",
  "gene": "UniProtKB:P01601"
}